actin capping protein of dynactin complex [GO:0005870] (cellular component) Definition: A heterodimer consisting of alpha and beta subunits that binds to and caps the barbed ends of actin filaments, nucleates the polymerization of actin monomers but does not sever actin filaments, and which is a part of the dynactin complex. Relationships: is a type of F-actin capping protein complex [GO:0008290]; BFO_0000050 dynactin complex [GO:0005869] References: PMID:18221362, PMID:18544499 Sources: GOC:jl